{
  "gene_name": "Voltage-dependent L-type calcium channel subunit alpha-1F",
  "term_label": "voltage-gated calcium channel complex",
  "gene_symbol": "CACNA1F",
  "gene": "UniProtKB:O60840",
  "term_id": "GO:0005891"
}